{
  "term_label": "regulation of actin cytoskeleton organization",
  "gene_symbol": "ARAP3",
  "gene_name": "Arf-GAP with Rho-GAP domain, ANK repeat and PH domain-containing protein 3",
  "gene": "UniProtKB:Q8WWN8",
  "term_id": "GO:0032956"
}